{
  "term_label": "dCMP deaminase activity",
  "gene": "UniProtKB:P32321",
  "gene_name": "Deoxycytidylate deaminase",
  "gene_symbol": "DCTD",
  "term_id": "GO:0004132"
}